{
  "gene": "UniProtKB:Q9NWF4",
  "gene_symbol": "SLC52A1",
  "term_label": "riboflavin transport",
  "term_id": "GO:0032218",
  "gene_name": "Solute carrier family 52, riboflavin transporter, member 1"
}